{
  "gene_symbol": "HSFX4",
  "term_label": "nucleus",
  "term_id": "GO:0005634",
  "gene": "UniProtKB:A0A1B0GTS1",
  "gene_name": "Heat shock transcription factor, X-linked member 4"
}